{
  "gene_name": "Guanine nucleotide-binding protein subunit beta-5",
  "gene_symbol": "GNB5",
  "term_id": "GO:0030159",
  "gene": "UniProtKB:O14775",
  "term_label": "signaling receptor complex adaptor activity"
}